{
  "term_id": "GO:0006357",
  "gene_name": "Aryl hydrocarbon receptor nuclear translocator 2",
  "gene_symbol": "ARNT2",
  "term_label": "regulation of transcription by RNA polymerase II",
  "gene": "UniProtKB:Q9HBZ2"
}